{
  "gene_name": "HORMA domain-containing protein 1",
  "gene_symbol": "HORMAD1",
  "term_label": "Unknown molecular function",
  "term_id": "UNKNOWN:0001",
  "gene": "UniProtKB:Q86X24"
}